{
  "gene": "UniProtKB:Q96BR9",
  "gene_name": "Zinc finger and BTB domain-containing protein 8A",
  "term_id": "UNKNOWN:0003",
  "term_label": "Unknown cellular component",
  "gene_symbol": "ZBTB8A"
}